regulation of seed development [GO:0080050] (BP) Definition: Any process that modulates the frequency, rate or extent of seed development. Subtypes: regulation of seed maturation [GO:2000034] Relationships: is a type of GO:0048580; is a type of GO:2000241; regulates seed development [GO:0048316] References: PMID:19141706